{
  "gene_name": "DNA dC-dU-editing enzyme APOBEC-3G",
  "term_label": "DNA cytosine deamination",
  "gene": "UniProtKB:Q9HC16",
  "gene_symbol": "APOBEC3G",
  "term_id": "GO:0070383"
}